{
  "term_label": "Unknown cellular component",
  "gene": "UniProtKB:O14960",
  "gene_symbol": "LECT2",
  "term_id": "UNKNOWN:0003",
  "gene_name": "Leukocyte cell-derived chemotaxin-2"
}